positive regulation of protein import into chloroplast stroma [GO:1904216] (biological process) Also known as: positive regulation of chloroplast stroma protein import, positive regulation of protein transport into chloroplast stroma, up regulation of chloroplast stroma protein import, up regulation of protein import into chloroplast stroma, up regulation of protein transport into chloroplast stroma, up-regulation of chloroplast stroma protein import, up-regulation of protein import into chloroplast stroma, up-regulation of protein transport into chloroplast stroma, upregulation of chloroplast stroma protein import, upregulation of protein import into chloroplast stroma, upregulation of protein transport into chloroplast stroma, activation of chloroplast stroma protein import, activation of protein import into chloroplast stroma, activation of protein transport into chloroplast stroma Definition: Any process that activates or increases the frequency, rate or extent of protein import into chloroplast stroma. References: PMID:25901327 Sources: GOC:TermGenie, GO_REF:0000058 Relationships: is a type of positive regulation of transmembrane transport [GO:0034764]; is a type of positive regulation of protein transport [GO:0051222]; is a type of regulation of protein import into chloroplast stroma [GO:1904215]; RO_0002213 protein import into chloroplast stroma [GO:0045037]